C2 domain binding [GO:0110036] (molecular function) References: PMID:24882364 Sources: GOC:sl Definition: Binding to the C2 domain of a protein, a protein structural domain involved in targeting proteins to cell membranes. Relationships: is a type of protein domain specific binding [GO:0019904]